phosphatidylinositol bisphosphate phosphatase activity [GO:0034593] (molecular function) Relationships: is a type of GO:0052866 Also known as: phosphatidyl-inositol-bisphosphate phosphatase activity, diphosphoinositide phosphatase activity, phosphatidylinositol-bisphosphatase activity, triphosphoinositide phosphatase activity, triphosphoinositide phosphomonoesterase activity Subtypes: phosphatidylinositol-3,4-bisphosphate phosphatase activity [GO:0106017], phosphatidylinositol-3,5-bisphosphate phosphatase activity [GO:0106018], GO:0106019 Definition: Catalysis of the reaction: 1-phosphatidyl-1D-myo-inositol bisphosphate + H2O = phosphatidylinositol phosphate + phosphate. Sources: GOC:mah